L(+)-tartrate dehydratase activity [GO:0008730] (molecular function) Also known as: (R,R)-tartrate hydro-lyase (oxaloacetate-forming), (R,R)-tartrate hydro-lyase activity, L-(+)-tartaric acid dehydratase activity, L-tartrate dehydratase activity, tartaric acid dehydrase activity, tartrate dehydratase activity Sources: EC:4.2.1.32, RHEA:15413 Relationships: is_a hydro-lyase activity [GO:0016836] Definition: Catalysis of the reaction: L-tartrate = H2O + oxaloacetate.